{
  "gene_symbol": "TRIM64C",
  "term_id": "GO:0045087",
  "gene": "UniProtKB:A6NLI5",
  "term_label": "innate immune response",
  "gene_name": "Tripartite motif-containing protein 64C"
}